{
  "gene": "UniProtKB:Q8IUE0",
  "gene_name": "Homeobox protein TGIF2LY",
  "term_label": "negative regulation of transcription by RNA polymerase II",
  "term_id": "GO:0000122",
  "gene_symbol": "TGIF2LY"
}